{
  "gene_name": "Placental protein 13-like",
  "term_label": "carbohydrate binding",
  "term_id": "GO:0030246",
  "gene_symbol": "LGALS14",
  "gene": "UniProtKB:Q8TCE9"
}